nucleoside:proton symporter activity [GO:0015506] (molecular function) Definition: Enables the transfer of a solute or solutes from one side of a membrane to the other according to the reaction: nucleoside(out) + H+(out) = nucleoside(in) + H+(in). Sources: TC:2.A.1.10.1, TC:2.A.41.1.1 Also known as: nucleoside:hydrogen ion symporter activity, nucleoside:hydrogen symporter activity, nucleoside permease activity Relationships: is a type of nucleoside transmembrane transporter activity [GO:0005337]; is a type of GO:0015295 Subtypes: GO:0015394, xanthosine:proton symporter activity [GO:0015537]